{
  "gene_symbol": "RGS4",
  "gene_name": "Regulator of G-protein signaling 4",
  "gene": "UniProtKB:P49798",
  "term_label": "cytoplasmic side of plasma membrane",
  "term_id": "GO:0009898"
}